{
  "gene": "UniProtKB:P57796",
  "gene_symbol": "CABP4",
  "term_id": "GO:0007601",
  "gene_name": "Calcium-binding protein 4",
  "term_label": "visual perception"
}